{
  "gene": "UniProtKB:Q9NUV7",
  "gene_name": "Serine palmitoyltransferase 3",
  "gene_symbol": "SPTLC3",
  "term_label": "sphingosine biosynthetic process",
  "term_id": "GO:0046512"
}